{
  "gene_symbol": "PIGV",
  "gene_name": "GPI mannosyltransferase 2",
  "gene": "UniProtKB:Q9NUD9",
  "term_id": "GO:0006506",
  "term_label": "GPI anchor biosynthetic process"
}